{
  "gene": "UniProtKB:O15318",
  "gene_name": "DNA-directed RNA polymerase III subunit RPC7",
  "term_label": "cell population proliferation",
  "term_id": "GO:0008283",
  "gene_symbol": "POLR3G"
}